{
  "term_label": "spermatogenesis",
  "gene_name": "Platelet-activating factor acetylhydrolase IB subunit alpha2",
  "term_id": "GO:0007283",
  "gene_symbol": "PAFAH1B2",
  "gene": "UniProtKB:P68402"
}